response to mitotic cell cycle checkpoint signaling [GO:0072414] (biological process) Subtypes: GO:0072432, response to mitotic G2 DNA damage checkpoint signaling [GO:0072435], GO:0072444, response to cell size control checkpoint signaling [GO:0072470], response to mitotic spindle checkpoint signaling [GO:0072476], GO:1990820 Definition: A process that occurs in response to signals generated as a result of mitotic cell cycle checkpoint signaling. Sources: GOC:mtg_cell_cycle Relationships: is a type of response to cell cycle checkpoint signaling [GO:0072396] Also known as: mitotic cell cycle checkpoint effector process, mitotic G2/M transition checkpoint effector process, mitotic cell cycle G1/S checkpoint effector process, response to mitotic G2/M transition checkpoint signal, response to mitotic cell cycle G1/S checkpoint signaling, response to signal involved in mitotic G2/M transition checkpoint, response to signal involved in mitotic cell cycle G1/S checkpoint, response to signal involved in mitotic cell cycle checkpoint